{
  "gene_symbol": "C16orf87",
  "gene": "UniProtKB:Q6PH81",
  "term_id": "UNKNOWN:0002",
  "gene_name": "UPF0547 protein C16orf87",
  "term_label": "Unknown biological process"
}